regulation of mitotic spindle checkpoint [GO:1903504] (biological process) References: PMID:23442800 Sources: GOC:TermGenie, GO_REF:0000058 Relationships: is a type of regulation of mitotic cell cycle [GO:0007346]; is_a regulation of spindle checkpoint [GO:0090231]; regulates mitotic spindle checkpoint signaling [GO:0071174] Definition: Any process that modulates the frequency, rate or extent of mitotic spindle checkpoint. Subtypes: regulation of mitotic cell cycle spindle assembly checkpoint [GO:0090266] Note: Note that this term should not be used for direct manual annotation as it should always be possible to specify the type of spindle checkpoint (assembly, orientation or Dma1-dependent). Also known as: regulation of mitotic cell cycle spindle checkpoint